{
  "gene_symbol": "KCNH2",
  "term_id": "GO:0086013",
  "gene_name": "Potassium voltage-gated channel subfamily H member 2",
  "gene": "UniProtKB:Q12809",
  "term_label": "membrane repolarization during cardiac muscle cell action potential"
}